{
  "gene": "UniProtKB:Q7RTV3",
  "term_id": "GO:0000978",
  "term_label": "RNA polymerase II cis-regulatory region sequence-specific DNA binding",
  "gene_name": "Zinc finger protein 367",
  "gene_symbol": "ZNF367"
}